transport across blood-brain barrier [GO:0150104] (BP) Definition: The directed movement of substances (e.g. macromolecules, small molecules, ions) through the blood-brain barrier. Subtypes: copper ion transport across blood-brain barrier [GO:0097716], GO:1990379, xenobiotic transport across blood-brain barrier [GO:1990962] References: PMID:29377008 Sources: GOC:aruk, GOC:bc Also known as: transport across BBB, transport across blood brain barrier Regulation: regulated by GO:0150200; positively regulated by GO:0150201; negatively regulated by GO:0150202 Relationships: is a type of vascular transport [GO:0010232]